N-acetylneuraminate biosynthetic process [GO:0046380] (biological process) Sources: ISBN:0198506732 Definition: The chemical reactions and pathways resulting in the formation of N-acetylneuraminate, the anion of 5-(acetylamino)-3,5-dideoxy-D-glycero-D-galacto-non-3-ulosonic acid. Relationships: is a type of N-acetylneuraminate metabolic process [GO:0006054]; is a type of amide biosynthetic process [GO:0043604]; is a type of amino sugar biosynthetic process [GO:0046349]; is a type of carboxylic acid biosynthetic process [GO:0046394] Also known as: N-acetylneuraminate anabolism, N-acetylneuraminate biosynthesis, N-acetylneuraminate formation, N-acetylneuraminate synthesis